{
  "term_id": "UNKNOWN:0003",
  "gene_name": "Modulator of apoptosis 1",
  "term_label": "Unknown cellular component",
  "gene": "UniProtKB:Q96BY2",
  "gene_symbol": "MOAP1"
}